vascular endothelial growth factor receptor signaling pathway involved in lymphatic endothelial cell fate commitment [GO:0060851] (biological process) Also known as: vascular endothelial growth factor receptor signalling pathway involved in lymphatic endothelial cell fate commitment Relationships: is a type of vascular endothelial growth factor receptor signaling pathway [GO:0048010]; is part of lymphatic endothelial cell fate commitment [GO:0060838] Sources: GOC:dph, GOC:sdb_2009, GOC:tb Definition: The series of molecular signals generated as a consequence of vascular endothelial growth factor receptor binding to one of its physiological ligands that contributes to the commitment of a venous endothelial cell to a lymphatic endothelial cell fate.